{
  "gene_symbol": "C19orf84",
  "gene": "UniProtKB:I3L1E1",
  "term_id": "UNKNOWN:0001",
  "gene_name": "Uncharacterized protein C19orf84",
  "term_label": "Unknown molecular function"
}